{
  "term_label": "external side of plasma membrane",
  "gene_name": "Atypical chemokine receptor 2",
  "gene_symbol": "ACKR2",
  "term_id": "GO:0009897",
  "gene": "UniProtKB:O00590"
}